{
  "gene": "UniProtKB:Q7LGC8",
  "term_id": "GO:0050650",
  "term_label": "chondroitin sulfate proteoglycan biosynthetic process",
  "gene_symbol": "CHST3",
  "gene_name": "Carbohydrate sulfotransferase 3"
}